{
  "gene": "UniProtKB:Q99661",
  "gene_symbol": "KIF2C",
  "term_id": "GO:0005874",
  "term_label": "microtubule",
  "gene_name": "Kinesin-like protein KIF2C"
}